{
  "gene_name": "Histone H2B type 1-L",
  "term_label": "chromatin organization",
  "gene_symbol": "H2BC13",
  "gene": "UniProtKB:Q99880",
  "term_id": "GO:0006325"
}